{
  "gene": "UniProtKB:Q15691",
  "gene_symbol": "MAPRE1",
  "gene_name": "Microtubule-associated protein RP_EB family member 1",
  "term_id": "GO:0031110",
  "term_label": "regulation of microtubule polymerization or depolymerization"
}